{
  "term_id": "UNKNOWN:0003",
  "gene": "UniProtKB:Q5VWK0",
  "term_label": "Unknown cellular component",
  "gene_symbol": "NBPF6",
  "gene_name": "Neuroblastoma breakpoint family member 6"
}